{
  "term_label": "promoter-specific chromatin binding",
  "term_id": "GO:1990841",
  "gene": "UniProtKB:P35226",
  "gene_symbol": "BMI1",
  "gene_name": "Polycomb complex protein BMI-1"
}